{
  "gene_symbol": "CFAP99",
  "term_label": "Unknown biological process",
  "term_id": "UNKNOWN:0002",
  "gene": "UniProtKB:D6REC4",
  "gene_name": "Cilia- and flagella-associated protein 99"
}